{
  "gene_symbol": "LOC112268384",
  "gene_name": "Olfactory receptor",
  "gene": "UniProtKB:A0A2R8YEH3",
  "term_id": "GO:0005886",
  "term_label": "plasma membrane"
}